{
  "term_label": "phototransduction",
  "term_id": "GO:0007602",
  "gene_symbol": "RGR",
  "gene_name": "RPE-retinal G protein-coupled receptor",
  "gene": "UniProtKB:P47804"
}